{
  "term_label": "Golgi apparatus",
  "gene": "UniProtKB:Q8WTX9",
  "gene_name": "Palmitoyltransferase ZDHHC1",
  "term_id": "GO:0005794",
  "gene_symbol": "ZDHHC1"
}